{
  "term_label": "regulation of short-term neuronal synaptic plasticity",
  "gene_symbol": "SYAP1",
  "term_id": "GO:0048172",
  "gene": "UniProtKB:Q96A49",
  "gene_name": "Synapse-associated protein 1"
}